{
  "gene_symbol": "AGT",
  "gene_name": "Angiotensinogen",
  "term_label": "angiotensin-activated signaling pathway",
  "term_id": "GO:0038166",
  "gene": "UniProtKB:P01019"
}